{
  "gene": "UniProtKB:Q07001",
  "term_label": "acetylcholine receptor activity",
  "term_id": "GO:0015464",
  "gene_symbol": "CHRND",
  "gene_name": "Acetylcholine receptor subunit delta"
}